{
  "term_id": "GO:0005615",
  "gene_symbol": "SERPINI2",
  "term_label": "extracellular space",
  "gene_name": "Serpin I2",
  "gene": "UniProtKB:O75830"
}